{
  "term_label": "cortical cytoskeleton organization",
  "gene_symbol": "RAC3",
  "gene": "UniProtKB:P60763",
  "gene_name": "Ras-related C3 botulinum toxin substrate 3",
  "term_id": "GO:0030865"
}